{
  "gene": "UniProtKB:Q9Y241",
  "term_label": "negative regulation of apoptotic process",
  "gene_name": "HIG1 domain family member 1A, mitochondrial",
  "gene_symbol": "HIGD1A",
  "term_id": "GO:0043066"
}